N-terminal protein amino acid acetylation [GO:0006474] (biological process) Relationships: is a type of protein acetylation [GO:0006473]; is a type of GO:0031365; is a type of protein maturation [GO:0051604] Definition: The acetylation of the N-terminal amino acid of proteins. Also known as: N(alpha)-terminal acetylation Sources: GOC:ai Subtypes: N-terminal peptidyl-aspartic acid acetylation [GO:0017190], N-terminal peptidyl-glutamine acetylation [GO:0017192], GO:0017196, N-terminal peptidyl-glutamic acid acetylation [GO:0018002], N-terminal peptidyl-lysine acetylation [GO:0018076]